{
  "gene_name": "Stromelysin-2",
  "term_id": "GO:0004222",
  "gene_symbol": "MMP10",
  "term_label": "metalloendopeptidase activity",
  "gene": "UniProtKB:P09238"
}